{
  "gene_symbol": "TNRC6B",
  "gene_name": "Trinucleotide repeat-containing gene 6B protein",
  "term_label": "Unknown molecular function",
  "term_id": "UNKNOWN:0001",
  "gene": "UniProtKB:Q9UPQ9"
}